dTDP-mannose biosynthetic process [GO:0019308] (biological process) Definition: The chemical reactions and pathways resulting in the formation of dTDP-mannose, a substance composed of mannose in glycosidic linkage with deoxyribosylthymine diphosphate. Also known as: dTDP-mannose anabolism, dTDP-mannose biosynthesis, dTDP-mannose formation, dTDP-mannose synthesis Sources: GOC:ai Relationships: is a type of GO:0009226